{
  "gene_symbol": "ZPBP2",
  "term_label": "acrosome assembly",
  "gene_name": "Zona pellucida-binding protein 2",
  "term_id": "GO:0001675",
  "gene": "UniProtKB:Q6X784"
}